UFM1 ligase activity [GO:0061666] (molecular function) Sources: GOC:dph Also known as: E3 Definition: Catalysis of the transfer of UFM1 to a substrate protein via the reaction X-UFM1 + S = X + S-UFM1, where X is either an E2 or E3 enzyme, the X-UFM1 linkage is a thioester bond, and the S-UFM1 linkage is an isopeptide bond between the C-terminal amino acid of UFM1 and the epsilon-amino group of lysine residues in the substrate. Relationships: is a type of GO:0061659; is a type of UFM1 transferase activity [GO:0071568]